{
  "term_id": "GO:0016492",
  "term_label": "G protein-coupled neurotensin receptor activity",
  "gene_symbol": "NTSR1",
  "gene_name": "Neurotensin receptor type 1",
  "gene": "UniProtKB:P30989"
}